regulation of renal phosphate excretion [GO:1903402] (biological process) Definition: Any process that modulates the frequency, rate or extent of renal phosphate excretion. Subtypes: GO:1903403, positive regulation of renal phosphate excretion [GO:1903404] Also known as: regulation of renal phosphate ion excretion Relationships: is a type of regulation of excretion [GO:0044062]; is a type of regulation of renal system process [GO:0098801]; regulates renal phosphate excretion [GO:0044722] References: PMID:8700837 Sources: GOC:TermGenie, GOC:pm, GO_REF:0000058